cytochrome c-heme linkage [GO:0018063] (biological process) Definition: The linkage of cytochromes and other heme proteins to heme. Sources: RESID:AA0134, RESID:AA0135 Relationships: is a type of GO:0017003; is a type of cytochrome complex assembly [GO:0017004] Also known as: cytochrome c-haem linkage